{
  "gene_name": "Thymosin beta-4",
  "term_id": "GO:0140311",
  "gene_symbol": "TMSB4X",
  "term_label": "protein sequestering activity",
  "gene": "UniProtKB:P62328"
}